{
  "term_label": "adherens junction",
  "gene_name": "Protein scribble homolog",
  "gene": "UniProtKB:Q14160",
  "gene_symbol": "SCRIB",
  "term_id": "GO:0005912"
}